excitatory chemical synaptic transmission [GO:0098976] (biological process) Definition: Synaptic transmission that results in an excitatory postsynaptic potential. Sources: GOC:dos Relationships: is a type of GO:0007268; has part excitatory postsynaptic potential [GO:0060079]